polytene chromosome chromocenter [GO:0005701] (CC) Sources: GOC:bf, ISBN:0120649012 Also known as: polytene chromosome chromocentre Definition: A region at which the centric regions of polytene chromosomes are joined together. Relationships: is a type of GO:0010369; is part of polytene chromosome [GO:0005700]